{
  "gene_symbol": "OBP2B",
  "term_label": "Unknown molecular function",
  "gene": "UniProtKB:Q9NPH6",
  "gene_name": "Odorant-binding protein 2b",
  "term_id": "UNKNOWN:0001"
}